{
  "term_id": "GO:0004175",
  "gene_name": "Proteasome subunit beta type-8",
  "gene_symbol": "PSMB8",
  "gene": "UniProtKB:P28062",
  "term_label": "endopeptidase activity"
}